{
  "gene_symbol": "EP400P1",
  "gene": "UniProtKB:Q6ZTU2",
  "gene_name": "Putative EP400-like protein",
  "term_id": "UNKNOWN:0001",
  "term_label": "Unknown molecular function"
}